eisosome filament [GO:0036286] (cellular component) Also known as: linear eisosome References: PMID:21900489, PMID:23722945 Sources: GOC:vw Definition: A filamentous cortical structure formed, in S. pombe, by the eisosome component Pil1. Relationships: is a type of protein-containing complex [GO:0032991]; is part of cortical cytoskeleton [GO:0030863]; is part of eisosome [GO:0032126]